{
  "gene": "UniProtKB:Q9HCH5",
  "gene_name": "Synaptotagmin-like protein 2",
  "gene_symbol": "SYTL2",
  "term_label": "plasma membrane",
  "term_id": "GO:0005886"
}